{
  "term_id": "GO:0005654",
  "term_label": "nucleoplasm",
  "gene": "UniProtKB:P31943",
  "gene_symbol": "HNRNPH1",
  "gene_name": "Heterogeneous nuclear ribonucleoprotein H"
}